symbiont-mediated suppression of host adaptive immune response [GO:0039504] (biological process) Subtypes: GO:0039588, symbiont-mediated suppression of host T-cell mediated immune response [GO:0052085], symbiont-mediated suppression of host B-cell mediated immune response [GO:0052086] Also known as: negative regulation of host adaptive immune response, negative regulation of host adaptive immunity, suppression of host acquired immune response, inhibition of host adaptive immune response by virus, suppression by virus of host adaptive immune response Relationships: is a type of symbiont-mediated suppression of host immune response [GO:0052562] Definition: A process by which a symbiont inhibits or disrupts the normal execution of the adaptive immune response of the host organism, an immune response based on directed amplification of specific receptors for antigen produced through a somatic diversification process, and allowing for enhanced response to subsequent exposures to the same antigen (immunological memory). Sources: GOC:add, GOC:bf, GOC:sp